positive regulation of actin filament-based movement [GO:1903116] (biological process) References: PMID:24798735 Sources: GOC:TermGenie, GO_REF:0000058 Subtypes: GO:0061874, positive regulation of cardiac muscle cell contraction [GO:0106134], positive regulation of apical constriction involved in ventral furrow formation [GO:0110074], positive regulation of muscle filament sliding [GO:1904114], positive regulation of myofibroblast contraction [GO:1904330] Definition: Any process that activates or increases the frequency, rate or extent of actin filament-based movement. Also known as: up regulation of actin filament-based movement, up-regulation of actin filament-based movement, upregulation of actin filament-based movement, activation of actin filament-based movement Relationships: is a type of positive regulation of cellular process [GO:0048522]; is a type of regulation of actin filament-based movement [GO:1903115]; RO_0002213 actin filament-based movement [GO:0030048]